{
  "gene_name": "4-hydroxyphenylpyruvate dioxygenase",
  "gene_symbol": "HPD",
  "term_id": "GO:0005789",
  "term_label": "endoplasmic reticulum membrane",
  "gene": "UniProtKB:P32754"
}